{
  "gene_symbol": "DCPS",
  "gene": "UniProtKB:Q96C86",
  "term_id": "GO:0005634",
  "gene_name": "m7GpppX diphosphatase",
  "term_label": "nucleus"
}